{
  "gene": "UniProtKB:Q8NDZ4",
  "term_label": "extracellular space",
  "term_id": "GO:0005615",
  "gene_name": "Divergent protein kinase domain 2A",
  "gene_symbol": "DIPK2A"
}